positive regulation of programmed cell death [GO:0043068] (biological process) Definition: Any process that activates or increases the frequency, rate or extent of programmed cell death, cell death resulting from activation of endogenous cellular processes. Subtypes: GO:0012502, positive regulation of plant-type hypersensitive response [GO:0034052], positive regulation of apoptotic process [GO:0043065], positive regulation of retinal cell programmed cell death [GO:0046670], positive regulation of killing of cells of another organism [GO:0051712], positive regulation of programmed necrotic cell death [GO:0062100], positive regulation of ferroptosis [GO:0160020], positive regulation of hydrogen peroxide-mediated programmed cell death [GO:1901300], positive regulation of autophagic cell death [GO:1904094], positive regulation of cornification [GO:1905717] Relationships: is a type of regulation of programmed cell death [GO:0043067]; is a type of positive regulation of cellular process [GO:0048522]; positively regulates programmed cell death [GO:0012501] Also known as: up regulation of programmed cell death, up-regulation of programmed cell death, upregulation of programmed cell death, activation of programmed cell death, positive regulation of non-apoptotic programmed cell death, stimulation of programmed cell death Sources: GOC:jl